{
  "gene": "UniProtKB:P78426",
  "term_id": "GO:0006357",
  "gene_symbol": "NKX6-1",
  "gene_name": "Homeobox protein Nkx-6.1",
  "term_label": "regulation of transcription by RNA polymerase II"
}